{
  "gene": "UniProtKB:Q8N7E2",
  "gene_name": "E3 ubiquitin-protein ligase CBLL2",
  "gene_symbol": "CBLL2",
  "term_id": "GO:0030155",
  "term_label": "regulation of cell adhesion"
}